{
  "term_id": "GO:0005579",
  "gene_name": "Complement component C9",
  "gene": "UniProtKB:P02748",
  "gene_symbol": "C9",
  "term_label": "membrane attack complex"
}